{
  "gene_symbol": "ADIRF",
  "term_id": "UNKNOWN:0001",
  "term_label": "Unknown molecular function",
  "gene": "UniProtKB:Q15847",
  "gene_name": "Adipogenesis regulatory factor"
}